{
  "gene_symbol": "MARCHF8",
  "gene_name": "E3 ubiquitin-protein ligase MARCHF8",
  "term_id": "GO:0005764",
  "term_label": "lysosome",
  "gene": "UniProtKB:Q5T0T0"
}